{
  "gene": "UniProtKB:P78344",
  "term_label": "mRNA binding",
  "term_id": "GO:0003729",
  "gene_symbol": "EIF4G2",
  "gene_name": "Eukaryotic translation initiation factor 4 gamma 2"
}